{
  "gene_name": "C-C motif chemokine 2",
  "gene": "UniProtKB:P13500",
  "term_id": "GO:0008009",
  "gene_symbol": "CCL2",
  "term_label": "chemokine activity"
}